{
  "gene": "UniProtKB:Q99758",
  "term_label": "ATPase-coupled transmembrane transporter activity",
  "gene_symbol": "ABCA3",
  "term_id": "GO:0042626",
  "gene_name": "Phospholipid-transporting ATPase ABCA3"
}